{
  "gene": "UniProtKB:Q6ZV65",
  "term_id": "GO:0045815",
  "term_label": "transcription initiation-coupled chromatin remodeling",
  "gene_name": "Protein FAM47E",
  "gene_symbol": "FAM47E"
}